apoptotic process [GO:0006915] (biological process) Definition: A programmed cell death process which begins when a cell receives an internal (e.g. DNA damage) or external signal (e.g. an extracellular death ligand), and proceeds through a series of biochemical events (signaling pathway phase) which trigger an execution phase. The execution phase is the last step of an apoptotic process, and is typically characterized by rounding-up of the cell, retraction of pseudopodes, reduction of cellular volume (pyknosis), chromatin condensation, nuclear fragmentation (karyorrhexis), plasma membrane blebbing and fragmentation of the cell into apoptotic bodies. When the execution phase is completed, the cell has died. References: PMID:18846107, PMID:21494263 Sources: GOC:cjm, GOC:dhl, GOC:ecd, GOC:go_curators, GOC:mtg_apoptosis Also known as: cell suicide, cellular suicide, apoptotic cell death, apoptotic programmed cell death, programmed cell death by apoptosis, activation of apoptosis, apoptosis, apoptosis signaling, apoptotic program, type I programmed cell death, apoptosis activator activity, caspase-dependent programmed cell death, commitment to apoptosis, induction of apoptosis, induction of apoptosis by p53, signaling (initiator) caspase activity Regulation: regulated by regulation of apoptotic process [GO:0042981]; positively regulated by GO:0043065; negatively regulated by GO:0043066 Relationships: is a type of programmed cell death [GO:0012501]; has part apoptotic signaling pathway [GO:0097190]; has part GO:0097194 Subtypes: inflammatory cell apoptotic process [GO:0006925], muscle cell apoptotic process [GO:0010657], myeloid cell apoptotic process [GO:0033028], glial cell apoptotic process [GO:0034349], anoikis [GO:0043276], fibroblast apoptotic process [GO:0044346], neuron apoptotic process [GO:0051402], apoptotic process in bone marrow cell [GO:0071839], leukocyte apoptotic process [GO:0071887], endothelial cell apoptotic process [GO:0072577], mesenchymal cell apoptotic process [GO:0097152], GO:0140208, melanocyte apoptotic process [GO:1902362], GO:1902489, GO:1902742, epithelial cell apoptotic process [GO:1904019], myofibroblast cell apoptotic process [GO:1904516], fat cell apoptotic process [GO:1904606], GO:1990009